{
  "gene_name": "Tetraspanin-9",
  "term_id": "GO:0005886",
  "gene_symbol": "TSPAN9",
  "term_label": "plasma membrane",
  "gene": "UniProtKB:O75954"
}